{
  "gene": "UniProtKB:Q86Y27",
  "gene_symbol": "BAGE5",
  "term_id": "UNKNOWN:0001",
  "term_label": "Unknown molecular function",
  "gene_name": "B melanoma antigen 5"
}